Rpd3L complex [GO:0033698] (cellular component) Definition: A histone deacetylase complex which deacetylates histones preferentially in promoter regions. Composed of a two copies of catalytic histone deacetylase subunit (S. pombe Clr6/ S. cerevisiae Rpd3p), an Sds-3 family protein (S. pombe /S. cerevisiae Sds3(p) ), two copies of SIN3 family co-repressor (S. pombe Pst1/ S. cerevisiae Sin3p, a WD repeat protein/ histone chaperone (S. pombe Prw1/ S. cerevisiae Ume1p), and a zf- PHD finger ( S. pombe Png2/ S. cerevisiae Pho23p), plus 4 additional subunits, and associated factors. Also known as: Clr6 histone deacetylase complex I/I', Clr6L complex, Rpd3C(L), Sin3L complex Relationships: is a type of GO:0070822 References: PMID:17450151 Sources: GOC:vw